protein tyrosine/serine/threonine phosphatase activity [GO:0008138] (molecular function) Also known as: dual-specificity protein phosphatase Definition: Catalysis of the reactions: protein serine + H2O = protein serine + phosphate; protein threonine phosphate + H2O = protein threonine + phosphate; and protein tyrosine phosphate + H2O = protein tyrosine + phosphate. Sources: GOC:mah Subtypes: JUN kinase phosphatase activity [GO:0008579], GO:0017017 Relationships: is a type of phosphoprotein phosphatase activity [GO:0004721]